{
  "gene_symbol": "AVIL",
  "gene": "UniProtKB:O75366",
  "term_label": "actin filament binding",
  "term_id": "GO:0051015",
  "gene_name": "Advillin"
}